{
  "gene_name": "Ras-related protein Rab-17",
  "term_label": "early endosome",
  "term_id": "GO:0005769",
  "gene_symbol": "RAB17",
  "gene": "UniProtKB:Q9H0T7"
}